{
  "gene_symbol": "LRRC69",
  "gene": "UniProtKB:Q6ZNQ3",
  "term_id": "UNKNOWN:0001",
  "term_label": "Unknown molecular function",
  "gene_name": "Leucine-rich repeat-containing protein 69"
}